rhombomere 4 structural organization [GO:0021662] (biological process) Sources: GOC:cls, GOC:dgh, GOC:dph, GOC:jid, GO_REF:0000021 Definition: The process that contributes to creating the structural organization of rhombomere 4. This process pertains to the physical shaping of a rudimentary structure. Rhombomeres are transverse segments of the developing rhombencephalon. Rhombomeres are lineage restricted, express different genes from one another, and adopt different developmental fates. Rhombomeres are numbered in an anterior to posterior order. Also known as: rhombomere 4 structural organisation Relationships: is a type of rhombomere structural organization [GO:0021595]; is part of rhombomere 4 morphogenesis [GO:0021661]